membrane tubulation [GO:0097749] (biological process) Subtypes: endosome membrane tubulation [GO:0097750] Sources: GOC:pr Relationships: is a type of membrane organization [GO:0061024] Definition: A membrane organization process resulting in the formation of a tubular projection. This may face inwardly (as in tubular membrane invaginations) or outwardly (as in endosomal tubules).